translation repressor activity [GO:0030371] (molecular function) Sources: GOC:ai, GOC:clt Relationships: is a type of GO:0045182; is part of negative regulation of translation [GO:0017148] Definition: Antagonizes ribosome-mediated translation of mRNA into a polypeptide. Subtypes: mRNA regulatory element binding translation repressor activity [GO:0000900], translation repressor activity, non-nucleic acid binding [GO:0000901], small RNA binding translational repressor activity [GO:0140764]